malonic acid transport [GO:1900752] (BP) Also known as: propanedioic acid transport, C3H4O4 transport, H2malo transport, HOOC-CH2-COOH transport Definition: The directed movement of a malonic acid into, out of or within a cell, or between cells, by means of some agent such as a transporter or pore. Subtypes: malonic acid transmembrane transport [GO:1901553] References: PMID:9128730, PMID:9573154 Sources: GOC:TermGenie Relationships: is a type of dicarboxylic acid transport [GO:0006835]